negative regulation of emodin biosynthetic process [GO:1900665] (biological process) Relationships: is a type of negative regulation of small molecule metabolic process [GO:0062014]; is a type of negative regulation of secondary metabolite biosynthetic process [GO:1900377]; is a type of regulation of emodin biosynthetic process [GO:1900664]; negatively regulates GO:1900575 Also known as: down regulation of emodin anabolism, down regulation of emodin biosynthesis, down regulation of emodin biosynthetic process, down regulation of emodin formation, down regulation of emodin synthesis, down-regulation of emodin anabolism, down-regulation of emodin biosynthesis, down-regulation of emodin biosynthetic process, down-regulation of emodin formation, down-regulation of emodin synthesis, downregulation of emodin anabolism, downregulation of emodin biosynthesis, downregulation of emodin biosynthetic process, downregulation of emodin formation, downregulation of emodin synthesis, inhibition of emodin anabolism, inhibition of emodin biosynthesis, inhibition of emodin formation, inhibition of emodin synthesis, negative regulation of emodin anabolism, negative regulation of emodin biosynthesis, negative regulation of emodin formation, negative regulation of emodin synthesis, inhibition of emodin biosynthetic process Sources: GOC:TermGenie, GOC:di Definition: Any process that stops, prevents or reduces the frequency, rate or extent of emodin biosynthetic process.